otolith mineralization [GO:0045299] (biological process) Definition: The precipitation of specific crystal forms of calcium carbonate with extracellular matrix proteins in the otolith organs of the vertebrate inner ear. Relationships: is_a GO:0031214; is part of otolith development [GO:0048840] References: PMID:15581873 Sources: GOC:dsf Subtypes: GO:0031173, GO:0031174